{
  "term_id": "GO:0001570",
  "gene": "UniProtKB:P35713",
  "gene_name": "Transcription factor SOX-18",
  "term_label": "vasculogenesis",
  "gene_symbol": "SOX18"
}